peptidyl-arginine modification [GO:0018195] (biological process) Sources: GOC:go_curators Subtypes: GO:0018109, GO:0018216, peptidyl-arginine hydroxylation [GO:0030961], peptidyl-arginine deglycation [GO:0036527] Relationships: is a type of peptidyl-amino acid modification [GO:0018193] Definition: The modification of peptidyl-arginine.